{
  "gene_symbol": "NOSTRIN",
  "gene": "UniProtKB:Q8IVI9",
  "term_label": "protein-macromolecule adaptor activity",
  "term_id": "GO:0030674",
  "gene_name": "Nostrin"
}